{
  "gene_symbol": "GABRA2",
  "gene_name": "Gamma-aminobutyric acid receptor subunit alpha-2",
  "gene": "UniProtKB:P47869",
  "term_label": "GABA-gated chloride ion channel activity",
  "term_id": "GO:0022851"
}